cell adhesion involved in retrograde extension [GO:0003392] (biological process) Definition: The attachment of a cell, either to another cell or to an underlying substrate such as the extracellular matrix that contributes to the process of retrograde extension. Subtypes: cell adhesion involved in dendrite retrograde extension [GO:0003394] Sources: GOC:ascb_2009, GOC:dph, GOC:tb Relationships: is a type of GO:0007155; is part of retrograde extension [GO:0003389]